{
  "gene_name": "Autophagy-related protein 9B",
  "gene_symbol": "ATG9B",
  "gene": "UniProtKB:Q674R7",
  "term_label": "protein localization to phagophore assembly site",
  "term_id": "GO:0034497"
}